{
  "term_label": "Unknown biological process",
  "gene": "UniProtKB:A8MRT5",
  "term_id": "UNKNOWN:0002",
  "gene_name": "Nuclear pore complex-interacting protein family member B5",
  "gene_symbol": "NPIPB5"
}